zona pellucida receptor complex [GO:0002199] (cellular component) Definition: A multisubunit complex comprising the chaperonin-containing T-complex and several other components involved in mediating sperm-oocyte Interaction. References: PMID:21880732 Sources: GOC:hjd Also known as: sperm protein complex I Relationships: is_a protein-containing complex [GO:0032991]; has part chaperonin-containing T-complex [GO:0005832]